{
  "gene_name": "Tryptophan 5-hydroxylase 2",
  "gene": "UniProtKB:Q8IWU9",
  "term_id": "UNKNOWN:0002",
  "gene_symbol": "TPH2",
  "term_label": "Unknown biological process"
}